{
  "gene": "UniProtKB:P49736",
  "gene_symbol": "MCM2",
  "term_id": "GO:0042555",
  "gene_name": "DNA replication licensing factor MCM2",
  "term_label": "MCM complex"
}